{
  "gene": "UniProtKB:A0A0A0MRZ9",
  "term_id": "UNKNOWN:0001",
  "gene_name": "Immunoglobulin lambda variable 5-52",
  "term_label": "Unknown molecular function",
  "gene_symbol": "IGLV5-52"
}